L-serine transmembrane transporter activity [GO:0015194] (molecular function) Also known as: L-serine transporter activity, serine transporter activity, L-serine permease activity, threonine/serine:sodium symporter activity Definition: Enables the transfer of L-serine from one side of a membrane to the other. L-serine is the L-enantiomer of 2-amino-3-hydroxypropanoic acid. Sources: GOC:ai, GOC:jsg, GOC:mah, GOC:mtg_transport Relationships: is a type of L-amino acid transmembrane transporter activity [GO:0015179]; is part of GO:0015825